{
  "gene_symbol": "ERO1A",
  "term_label": "protein-disulfide reductase activity",
  "gene_name": "ERO1-like protein alpha",
  "gene": "UniProtKB:Q96HE7",
  "term_id": "GO:0015035"
}